intracellular aspartate homeostasis [GO:0090459] (biological process) Sources: GOC:tb Also known as: aspartate homeostasis, cellular aspartate homeostasis Definition: A homeostatic process involved in the maintenance of a steady state level of aspartate within a cell. Relationships: is_a intracellular amino acid homeostasis [GO:0080144]